positive regulation of focal adhesion assembly [GO:0051894] (biological process) Sources: GOC:ai Definition: Any process that activates or increases the frequency, rate or extent of focal adhesion assembly, the establishment and maturation of focal adhesions. Relationships: is a type of positive regulation of cell-matrix adhesion [GO:0001954]; is a type of regulation of focal adhesion assembly [GO:0051893]; is a type of positive regulation of cell-substrate junction organization [GO:0150117]; is a type of positive regulation of cell junction assembly [GO:1901890]; RO_0002213 GO:0048041 Also known as: up regulation of focal adhesion formation, up-regulation of focal adhesion formation, upregulation of focal adhesion formation, activation of focal adhesion formation, stimulation of focal adhesion formation